{
  "term_id": "UNKNOWN:0001",
  "gene": "UniProtKB:Q8N9W5",
  "gene_symbol": "DNAAF3",
  "gene_name": "Dynein axonemal assembly factor 3",
  "term_label": "Unknown molecular function"
}